{
  "gene_symbol": "ZMIZ1",
  "gene_name": "Zinc finger MIZ domain-containing protein 1",
  "term_id": "GO:0006357",
  "gene": "UniProtKB:Q9ULJ6",
  "term_label": "regulation of transcription by RNA polymerase II"
}